olefin metabolic process [GO:1900673] (biological process) Subtypes: GO:0009692, propylene metabolic process [GO:0018964], alkene catabolic process [GO:0043451], GO:0043611, limonene catabolic process [GO:0046251], olefin biosynthetic process [GO:1900674], octadecene metabolic process [GO:1900681], GO:1900876, (Z)-nonadeca-1,14-diene metabolic process [GO:1900878], 18-methylnonadec-1-ene metabolic process [GO:1900880], 17-methylnonadec-1-ene metabolic process [GO:1900882], (-)-exo-alpha-bergamotene catabolic process [GO:1901939] Sources: GOC:TermGenie, GOC:mengo_curators Relationships: is a type of hydrocarbon metabolic process [GO:0120252]; is a type of olefinic compound metabolic process [GO:0120254] Also known as: olefin metabolism Definition: The chemical reactions and pathways involving olefin.